{
  "gene": "UniProtKB:P51817",
  "gene_name": "cAMP-dependent protein kinase catalytic subunit PRKX",
  "term_label": "cytosol",
  "term_id": "GO:0005829",
  "gene_symbol": "PRKX"
}